epithelial cell differentiation involved in mammary gland alveolus development [GO:0061030] (biological process) Definition: The process in which a relatively unspecialized epithelial cell becomes a more specialized epithelial cell of the mammary gland alveolus. Relationships: is a type of mammary gland epithelial cell differentiation [GO:0060644]; is part of mammary gland alveolus development [GO:0060749] Sources: GOC:dph, GOC:yaf